{
  "gene": "UniProtKB:P00441",
  "gene_name": "Superoxide dismutase [Cu-Zn]",
  "term_label": "peroxisome",
  "gene_symbol": "SOD1",
  "term_id": "GO:0005777"
}